{
  "term_label": "Unknown cellular component",
  "gene_symbol": "SOWAHC",
  "term_id": "UNKNOWN:0003",
  "gene": "UniProtKB:Q53LP3",
  "gene_name": "Ankyrin repeat domain-containing protein SOWAHC"
}